phosphatidylserine decarboxylase activity [GO:0004609] (molecular function) Relationships: is_a carboxy-lyase activity [GO:0016831] Definition: Catalysis of the reaction: H+ + phosphatidyl-L-serine = CO2 + phosphatidylethanolamine. Also known as: PS decarboxylase activity, phosphatidyl-L-serine carboxy-lyase (phosphatidylethanolamine-forming), phosphatidyl-L-serine carboxy-lyase activity Sources: EC:4.1.1.65, RHEA:20828